{
  "gene_symbol": "MAS1",
  "gene": "UniProtKB:P04201",
  "term_id": "GO:0001595",
  "term_label": "angiotensin receptor activity",
  "gene_name": "Proto-oncogene Mas"
}